{
  "term_id": "GO:0005343",
  "term_label": "organic acid:sodium symporter activity",
  "gene_name": "Sodium-coupled monocarboxylate transporter 1",
  "gene": "UniProtKB:Q8N695",
  "gene_symbol": "SLC5A8"
}